{
  "gene_symbol": "CT45A1",
  "gene": "UniProtKB:Q5HYN5",
  "gene_name": "Cancer_testis antigen family 45 member A1",
  "term_id": "UNKNOWN:0002",
  "term_label": "Unknown biological process"
}